intrinsic apoptotic signaling pathway [GO:0097193] (biological process) Subtypes: intrinsic apoptotic signaling pathway in response to osmotic stress [GO:0008627], intrinsic apoptotic signaling pathway in response to DNA damage [GO:0008630], intrinsic apoptotic signaling pathway in response to oxidative stress [GO:0008631], GO:0070059, intrinsic apoptotic signaling pathway by p53 class mediator [GO:0072332], intrinsic apoptotic signaling pathway in response to hypoxia [GO:1990144], intrinsic apoptotic signaling pathway in response to nitrosative stress [GO:1990442] Note: The signals that start intrinsic apoptosis may come from extracellular sources (e.g. oxidative stress, UV exposure), but the reception of the signal and thus the signaling pathway start inside the cell (as a result of DNA damage, redox imbalance, etc.). Examples are ZPR9 (ZNF622) and ASK1 (MAP3K5) (UniProt symbols Q969S3 and Q99683) in PMID:21771788. A diagram of the intrinsic apoptotic pathway including examples of molecular players can be found in Figure 2 in PMID:21760595. Relationships: is a type of intracellular signal transduction [GO:0035556]; is a type of GO:0097190 Regulation: regulated by regulation of intrinsic apoptotic signaling pathway [GO:2001242]; negatively regulated by negative regulation of intrinsic apoptotic signaling pathway [GO:2001243]; positively regulated by positive regulation of intrinsic apoptotic signaling pathway [GO:2001244] Also known as: intrinsic apoptotic pathway, intrinsic apoptotic signalling pathway, mitochondrial-mediated apoptotic pathway, intrinsic apoptosis, induction of apoptosis by intracellular signals References: PMID:11919192, PMID:17340152, PMID:18852119 Sources: GOC:mtg_apoptosis, GOC:yaf Definition: The series of molecular signals in which an intracellular signal is conveyed to trigger the apoptotic death of a cell. The pathway starts with reception of an intracellular signal (e.g. DNA damage, endoplasmic reticulum stress, oxidative stress etc.), and ends when the execution phase of apoptosis is triggered. The intrinsic apoptotic signaling pathway is crucially regulated by permeabilization of the mitochondrial outer membrane (MOMP).